{
  "gene_name": "Cytochrome P450 11B1, mitochondrial",
  "term_label": "steroid 11-beta-monooxygenase activity",
  "term_id": "GO:0004507",
  "gene_symbol": "CYP11B1",
  "gene": "UniProtKB:P15538"
}